{
  "term_id": "GO:0031267",
  "term_label": "small GTPase binding",
  "gene_name": "Kinetochore-associated protein 1",
  "gene_symbol": "KNTC1",
  "gene": "UniProtKB:P50748"
}